actin monomer sequestering activity [GO:0003788] (molecular function) Relationships: is a type of protein sequestering activity [GO:0140311]; BFO_0000051 actin monomer binding [GO:0003785] Definition: Binding to an actin monomer to prevent it from interacting with other partners or to inhibit its localization to the area of the cell or complex where it is active. References: PMID:11274401, PMID:1447300